anterior lateral line nerve glial cell differentiation [GO:0048913] (BP) References: PMID:15832385 Definition: The process in which a relatively unspecialized cell acquires specialized features of a glial cell in the anterior lateral line nerve. Relationships: is a type of GO:0048895; is part of anterior lateral line nerve development [GO:0048909]